{
  "term_label": "cyclin-dependent protein serine/threonine kinase activator activity",
  "gene_name": "Cyclin-K",
  "term_id": "GO:0061575",
  "gene_symbol": "CCNK",
  "gene": "UniProtKB:O75909"
}